(+)-kotanin biosynthetic process [GO:1900596] (biological process) Regulation: regulated by regulation of (+)-kotanin biosynthetic process [GO:1900692]; negatively regulated by GO:1900693; positively regulated by positive regulation of (+)-kotanin biosynthetic process [GO:1900694] Also known as: (+)-kotanin anabolism, (+)-kotanin biosynthesis, (+)-kotanin formation, (+)-kotanin synthesis Definition: The chemical reactions and pathways resulting in the formation of (+)-kotanin. Sources: GOC:TermGenie, GOC:di Relationships: is a type of GO:0044550